{
  "gene_name": "Chromodomain Y-like protein",
  "term_id": "GO:0062072",
  "gene_symbol": "CDYL",
  "term_label": "histone H3K9me2/3 reader activity",
  "gene": "UniProtKB:Q9Y232"
}